{
  "gene_name": "Bridge-like lipid transfer protein family member 1",
  "gene": "UniProtKB:Q2LD37",
  "term_id": "UNKNOWN:0003",
  "term_label": "Unknown cellular component",
  "gene_symbol": "BLTP1"
}